{
  "term_id": "GO:0005615",
  "gene_symbol": "CREG2",
  "gene_name": "Protein CREG2",
  "term_label": "extracellular space",
  "gene": "UniProtKB:Q8IUH2"
}